{
  "term_label": "Unknown biological process",
  "gene": "UniProtKB:Q9H330",
  "gene_name": "Transmembrane protein 245",
  "gene_symbol": "TMEM245",
  "term_id": "UNKNOWN:0002"
}